{
  "term_id": "GO:0005815",
  "gene_symbol": "CCNB1",
  "gene": "UniProtKB:P14635",
  "term_label": "microtubule organizing center",
  "gene_name": "G2_mitotic-specific cyclin-B1"
}